{
  "term_id": "GO:0004596",
  "gene_name": "N-alpha-acetyltransferase 50",
  "gene": "UniProtKB:Q9GZZ1",
  "gene_symbol": "NAA50",
  "term_label": "protein-N-terminal amino-acid acetyltransferase activity"
}